DNA-deoxyinosine glycosylase activity [GO:0033958] (molecular function) Also known as: DNA(hypoxanthine) glycohydrolase activity, DNA-deoxyinosine deoxyribohydrolase activity, DNA-deoxyinosine glycosidase activity, deoxyribonucleic acid glycosylase activity, hypoxanthine-DNA glycosylase activity Sources: EC:3.2.2.15 Relationships: is a type of GO:0016799; is a type of catalytic activity, acting on DNA [GO:0140097] Definition: Catalysis of the hydrolysis of DNA and polynucleotides, releasing free hypoxanthine.